{
  "term_label": "G-protein beta-subunit binding",
  "gene_name": "Putative guanine nucleotide-binding protein G(I)_G(S)_G(O) subunit gamma-14",
  "term_id": "GO:0031681",
  "gene": "UniProtKB:A0A1W2PPG7",
  "gene_symbol": "GNG14"
}